{
  "gene_symbol": "OR10G4",
  "term_id": "GO:0050911",
  "gene": "UniProtKB:Q8NGN3",
  "gene_name": "Olfactory receptor 10G4",
  "term_label": "detection of chemical stimulus involved in sensory perception of smell"
}